{
  "gene_symbol": "RTL4",
  "term_label": "Unknown molecular function",
  "gene_name": "Retrotransposon Gag-like protein 4",
  "term_id": "UNKNOWN:0001",
  "gene": "UniProtKB:Q6ZR62"
}